{
  "term_label": "mitochondrial large ribosomal subunit",
  "term_id": "GO:0005762",
  "gene_name": "Large ribosomal subunit protein mL43",
  "gene_symbol": "MRPL43",
  "gene": "UniProtKB:Q8N983"
}